{
  "gene_name": "Signal transducer and activator of transcription 6",
  "gene_symbol": "STAT6",
  "gene": "UniProtKB:P42226",
  "term_id": "GO:0006357",
  "term_label": "regulation of transcription by RNA polymerase II"
}